{
  "gene": "UniProtKB:P0DP74",
  "gene_symbol": "DEFB130A",
  "gene_name": "Beta-defensin 130A",
  "term_label": "CCR6 chemokine receptor binding",
  "term_id": "GO:0031731"
}